positive regulation of turning behavior involved in mating [GO:0061095] (biological process) Relationships: is a type of regulation of turning behavior involved in mating [GO:0061094]; is_a positive regulation of male mating behavior [GO:1902437]; positively regulates turning behavior involved in mating [GO:0034607] Sources: GOC:dph, GOC:tb Definition: Any process that increases the rate, frequency or extent of turning behavior involved in mating. Turning behavior is the sharp ventral turn performed by the male as he approaches either the hermaphrodite head or tail, whilst trying to locate his partner's vulva. Turning occurs via a sharp ventral coil of the male's tail.